{
  "gene": "UniProtKB:Q96NI8",
  "gene_name": "Zinc finger protein 570",
  "gene_symbol": "ZNF570",
  "term_label": "DNA-binding transcription factor activity, RNA polymerase II-specific",
  "term_id": "GO:0000981"
}